secretory IgA immunoglobulin complex [GO:0071751] (cellular component) Relationships: is_a polymeric IgA immunoglobulin complex [GO:0071749] Also known as: sIgA antibody, secretory IgA antibody, sIgA1 antibody References: PMID:16362985 Sources: GOC:add, ISBN:0781765196 Definition: A polymeric IgA immunoglobulin complex that is complexed with one chain of secretory component (SC). Polymeric IgA is present in mucosal areas, having been transported via a transcytosis mechanism in mucosal epithelial cells relying on the polymeric Ig receptor, a portion of which then remains bound to the polymeric IgA as secretory component. Subtypes: secretory dimeric IgA immunoglobulin complex [GO:0071752] Note: Note that an IgA immunoglobulin complex has the function of antigen binding if a suitable antigen is available. In human only the IgA1 isotype in the polymeric form is capable of becoming secretory IgA.